carnitine catabolic process [GO:0042413] (biological process) Sources: GOC:jl, ISBN:0198506732 Also known as: carnitine breakdown, carnitine catabolism, carnitine degradation, vitamin Bt catabolic process, vitamin Bt catabolism Definition: The chemical reactions and pathways resulting in the breakdown of carnitine (hydroxy-trimethyl aminobutyric acid), a compound that participates in the transfer of acyl groups across the inner mitochondrial membrane. Relationships: is a type of amino-acid betaine catabolic process [GO:0006579]; is a type of carnitine metabolic process [GO:0009437]